parahippocampal gyrus development [GO:0021770] (biological process) Definition: The progression of the parahippocampal gyrus over time from its initial formation until its mature state. The parahippocampal gyrus is a ridge in the cerebral cortex. Also known as: hippocampal gyrus development Sources: GOC:cls, GOC:dgh, GOC:dph, GOC:jid, GO_REF:0000021 Relationships: is a type of anatomical structure development [GO:0048856]; is part of GO:0021761